{
  "term_label": "cytoplasm",
  "term_id": "GO:0005737",
  "gene_symbol": "PRDM1",
  "gene": "UniProtKB:O75626",
  "gene_name": "PR domain zinc finger protein 1"
}